{
  "gene_symbol": "FAM83E",
  "gene": "UniProtKB:Q2M2I3",
  "term_label": "signal transduction",
  "term_id": "GO:0007165",
  "gene_name": "Protein FAM83E"
}